{
  "gene_symbol": "NUS1",
  "gene_name": "Dehydrodolichyl diphosphate synthase complex subunit NUS1",
  "gene": "UniProtKB:Q96E22",
  "term_label": "endoplasmic reticulum membrane",
  "term_id": "GO:0005789"
}